{
  "gene": "UniProtKB:Q96L91",
  "gene_symbol": "EP400",
  "term_label": "DNA repair",
  "term_id": "GO:0006281",
  "gene_name": "E1A-binding protein p400"
}